regulation of metallopeptidase activity [GO:1905048] (biological process) Definition: Any process that modulates the frequency, rate or extent of metallopeptidase activity. Subtypes: negative regulation of metallopeptidase activity [GO:1905049], positive regulation of metallopeptidase activity [GO:1905050] References: PMID:26473732 Sources: GOC:TermGenie, GO_REF:0000059 Also known as: regulation of metalloprotease activity, regulation of metalloproteinase activity Relationships: is a type of regulation of peptidase activity [GO:0052547]; regulates GO:0008237